{
  "term_id": "GO:0045505",
  "term_label": "dynein intermediate chain binding",
  "gene_name": "Dynein light chain Tctex-type 1",
  "gene": "UniProtKB:P63172",
  "gene_symbol": "DYNLT1"
}